taste bud formation [GO:0061195] (biological process) Relationships: is a type of GO:0048646; is part of GO:0061194 Sources: GOC:dph Definition: The developmental process pertaining to the initial formation of the taste bud from unspecified parts. The taste bud is a specialized area of the tongue that contains taste receptors.